{
  "gene_symbol": "CXCL13",
  "gene_name": "C-X-C motif chemokine 13",
  "gene": "UniProtKB:O43927",
  "term_label": "chemokine activity",
  "term_id": "GO:0008009"
}